{
  "gene": "UniProtKB:Q9Y6J8",
  "gene_symbol": "STYXL1",
  "term_id": "GO:0001691",
  "term_label": "pseudophosphatase activity",
  "gene_name": "Serine_threonine_tyrosine-interacting-like protein 1"
}